{
  "gene": "UniProtKB:P20929",
  "gene_symbol": "NEB",
  "gene_name": "Nebulin",
  "term_id": "GO:0071691",
  "term_label": "cardiac muscle thin filament assembly"
}